{
  "gene": "UniProtKB:P42892",
  "term_label": "metalloendopeptidase activity",
  "gene_symbol": "ECE1",
  "gene_name": "Endothelin-converting enzyme 1",
  "term_id": "GO:0004222"
}